negative regulation of cell adhesion involved in sprouting angiogenesis [GO:0106089] (biological process) Relationships: is a type of GO:0007162; is a type of GO:0106088; is a type of negative regulation of sprouting angiogenesis [GO:1903671]; negatively regulates cell adhesion involved in sprouting angiogenesis [GO:0120078] References: PMID:24177325 Sources: GOC:BHF, GOC:BHF_miRNA, GOC:rph Definition: Any process that stops, prevents or reduces the frequency, rate or extent of cell adhesion involved in sprouting angiogenesis.